response to manganese ion starvation [GO:0090551] (biological process) Definition: Any process that results in a change in state or activity of a cell or an organism (in terms of movement, secretion, enzyme production, gene expression, etc.) as a result of a starvation stimulus, deprivation of manganese. Sources: GOC:tair_curators Relationships: is a type of response to metal ion starvation [GO:0180055]